{
  "gene": "UniProtKB:Q9Y4C4",
  "term_label": "inflammatory response",
  "gene_name": "Malignant fibrous histiocytoma-amplified sequence 1",
  "gene_symbol": "MFHAS1",
  "term_id": "GO:0006954"
}